{
  "gene_name": "Aquaporin-11",
  "gene_symbol": "AQP11",
  "gene": "UniProtKB:Q8NBQ7",
  "term_id": "GO:0005737",
  "term_label": "cytoplasm"
}